tetraterpenoid catabolic process [GO:0016110] (biological process) Subtypes: carotenoid catabolic process [GO:0016118] Relationships: is a type of terpenoid catabolic process [GO:0016115] Sources: GOC:go_curators Also known as: tetraterpenoid breakdown, tetraterpenoid catabolism, tetraterpenoid degradation, tetraterpene catabolic process, tetraterpene catabolism Definition: The chemical reactions and pathways resulting in the breakdown of tetraterpenoid compounds, terpenoids with eight isoprene units.